{
  "gene_symbol": "KLK12",
  "term_label": "protein maturation",
  "gene": "UniProtKB:Q9UKR0",
  "gene_name": "Kallikrein-12",
  "term_id": "GO:0051604"
}